negative regulation of endocardial cushion to mesenchymal transition involved in heart valve formation [GO:2000801] (biological process) Sources: GOC:BHF Definition: Any process that stops, prevents or reduces the frequency, rate or extent of endocardial cushion to mesenchymal transition involved in heart valve formation. Relationships: is a type of GO:0140050; is a type of regulation of endocardial cushion to mesenchymal transition involved in heart valve formation [GO:2000800]; RO_0002212 endocardial cushion to mesenchymal transition involved in heart valve formation [GO:0003199] Also known as: negative regulation of endocardial cushion to mesenchymal transition involved in valve formation